{
  "gene_name": "Olfactory receptor 1G1",
  "term_label": "olfactory receptor activity",
  "gene_symbol": "OR1G1",
  "gene": "UniProtKB:P47890",
  "term_id": "GO:0004984"
}